{
  "term_id": "GO:0005829",
  "gene": "UniProtKB:Q01415",
  "gene_name": "N-acetylgalactosamine kinase",
  "gene_symbol": "GALK2",
  "term_label": "cytosol"
}